{
  "gene_name": "Lysozyme C",
  "term_id": "GO:0005615",
  "gene": "UniProtKB:P61626",
  "term_label": "extracellular space",
  "gene_symbol": "LYZ"
}